{
  "term_id": "GO:0030674",
  "term_label": "protein-macromolecule adaptor activity",
  "gene_name": "Telethonin",
  "gene": "UniProtKB:O15273",
  "gene_symbol": "TCAP"
}